nuclear RNA surveillance [GO:0071027] (biological process) Subtypes: nuclear mRNA surveillance [GO:0071028], nuclear polyadenylation-dependent rRNA catabolic process [GO:0071035], nuclear polyadenylation-dependent snoRNA catabolic process [GO:0071036], nuclear polyadenylation-dependent snRNA catabolic process [GO:0071037], TRAMP-dependent tRNA surveillance pathway [GO:0071038], nuclear polyadenylation-dependent CUT catabolic process [GO:0071039], antisense RNA transcript catabolic process [GO:0071041], GO:0071046, RNA polymerase II transcription initiation surveillance [GO:0160240], nuclear lncRNA surveillance [GO:0180036] Relationships: is a type of GO:0071025; occurs in nucleus [GO:0005634] Definition: A process that identifies and degrades defective or aberrant RNAs within the nucleus. Also known as: nuclear RNA quality control, nuclear aberrant RNA catabolic process References: PMID:18644474 Sources: GOC:dgf, GOC:krc